positive regulation of chemotaxis to arachidonate [GO:1904554] (biological process) Definition: Any process that activates or increases the frequency, rate or extent of chemotaxis to arachidonic acid. Relationships: is a type of GO:0050921; is a type of regulation of chemotaxis to arachidonate [GO:1904552]; positively regulates chemotaxis to arachidonate [GO:0034670] References: PMID:16382163 Sources: GOC:TermGenie, GO_REF:0000058 Also known as: positive regulation of chemotaxis to arachidonic acid, up regulation of chemotaxis to arachidonic acid, up-regulation of chemotaxis to arachidonic acid, upregulation of chemotaxis to arachidonic acid, activation of chemotaxis to arachidonic acid